chromo shadow domain binding [GO:0070087] (molecular function) Relationships: is a type of protein domain specific binding [GO:0019904] Also known as: chromoshadow domain binding Definition: Binding to a chromo shadow domain, a protein domain that is distantly related, and found in association with, the chromo domain. References: PMID:7667093 Sources: GOC:BHF, GOC:vk, InterPro:IPR008251